{
  "gene_name": "Zinc finger protein 335",
  "gene_symbol": "ZNF335",
  "term_id": "GO:0050769",
  "term_label": "positive regulation of neurogenesis",
  "gene": "UniProtKB:Q9H4Z2"
}